{
  "term_label": "Unknown molecular function",
  "term_id": "UNKNOWN:0001",
  "gene_name": "Mitochondrial coiled-coil domain protein 1",
  "gene": "UniProtKB:P59942",
  "gene_symbol": "MCCD1"
}